succinate:fumarate antiporter activity [GO:0005469] (molecular function) Sources: TC:2.A.29.13.1 Definition: Enables the transfer of a solute or solutes from one side of a membrane to the other according to the reaction: succinate(out) + fumarate(in) = succinate(in) + fumarate(out). Relationships: is a type of fumarate transmembrane transporter activity [GO:0015138]; is a type of succinate transmembrane transporter activity [GO:0015141]; is a type of antiporter activity [GO:0015297]